luminal surveillance complex [GO:0034099] (cellular component) Definition: A multiprotein complex that recognizes ERAD-luminal misfolded substrates and brings them to the ubiquitination/extraction machinery. In yeast, this complex consists of Yos9p, Kar2p and Hrd3p proteins. References: PMID:16873065 Relationships: is_a GO:0140534; BFO_0000050 endoplasmic reticulum lumen [GO:0005788]